{
  "gene": "UniProtKB:Q05932",
  "gene_symbol": "FPGS",
  "gene_name": "Folylpolyglutamate synthase, mitochondrial",
  "term_label": "mitochondrion",
  "term_id": "GO:0005739"
}